oxaloacetase activity [GO:0030603] (molecular function) Definition: Catalysis of the reaction: H2O + oxaloacetate = acetate + H+ + oxalate. Relationships: is a type of hydrolase activity, acting on acid carbon-carbon bonds, in ketonic substances [GO:0016823] Also known as: oxalacetic hydrolase activity, oxaloacetate acetylhydrolase activity Sources: EC:3.7.1.1, RHEA:24432